regulation of mitophagy [GO:1901524] (biological process) Subtypes: negative regulation of mitophagy [GO:1901525], GO:1901526, regulation of type 2 mitophagy [GO:1905089] Definition: Any process that modulates the frequency, rate or extent of macromitophagy. Also known as: regulation of macromitophagy Sources: GOC:TermGenie Relationships: is_a regulation of macroautophagy [GO:0016241]; is a type of regulation of autophagy of mitochondrion [GO:1903146]; RO_0002211 mitophagy [GO:0000423]